{
  "term_id": "GO:0007165",
  "gene": "UniProtKB:P31947",
  "gene_name": "14-3-3 protein sigma",
  "gene_symbol": "SFN",
  "term_label": "signal transduction"
}